{
  "term_label": "defense response to virus",
  "term_id": "GO:0051607",
  "gene": "UniProtKB:Q9NR97",
  "gene_name": "Toll-like receptor 8",
  "gene_symbol": "TLR8"
}